{
  "gene_name": "Protein Mis18-alpha",
  "term_id": "UNKNOWN:0001",
  "gene": "UniProtKB:Q9NYP9",
  "gene_symbol": "MIS18A",
  "term_label": "Unknown molecular function"
}